{
  "gene_name": "Large ribosomal subunit protein uL16",
  "gene_symbol": "RPL10",
  "term_id": "GO:0006412",
  "term_label": "translation",
  "gene": "UniProtKB:P27635"
}